{
  "term_id": "GO:0061630",
  "gene": "UniProtKB:Q96PU5",
  "gene_name": "E3 ubiquitin-protein ligase NEDD4-like",
  "gene_symbol": "NEDD4L",
  "term_label": "ubiquitin protein ligase activity"
}